septin ring disassembly [GO:0031107] (biological process) Relationships: is a type of septin ring organization [GO:0031106]; is a type of organelle disassembly [GO:1903008] Sources: GOC:mah Definition: The controlled breakdown of a septin ring.